vancomycin biosynthetic process [GO:0033072] (biological process) Relationships: is a type of nonribosomal peptide biosynthetic process [GO:0019184]; is a type of GO:0030651; is a type of carbohydrate derivative biosynthetic process [GO:1901137] Sources: GOC:mah Also known as: vancomycin anabolism, vancomycin biosynthesis, vancomycin formation, vancomycin synthesis Definition: The chemical reactions and pathways leading to the formation of vancomycin, (3S,6R,7R,11R,23S,26S,30aS,36R,38aR)-44-[2-O-(3-amino-2,3,6-trideoxy-3-C-methyl-alpha-L-lyxo-hexopyranosyl)-beta-D-glucopyranosyloxy]-3-(carbamoylmethyl)-10,19-dichloro-2,3,4,5,6,7,23,25,26,36,37,38,38a-tetradecahydro-7,22,28,30,32-pentahydroxy-6-(N-methyl-D-leucyl)-2,5,24,38,39-pentaoxo-1H,22H-23,36-(epiminomethano)-8,11:18,21-dietheno-13,16:31,35-di(metheno)[1,6,9]oxadiazacyclohexadecino[4,5-m][10,2,16]benzoxadiazacyclotetracosine-26-carboxylic acid, a complex glycopeptide from Streptomyces orientalis that inhibits a specific step in the synthesis of the peptidoglycan layer in Gram-positive bacteria.